{
  "gene_symbol": "TRIM67",
  "term_label": "Unknown biological process",
  "gene_name": "Tripartite motif-containing protein 67",
  "gene": "UniProtKB:Q6ZTA4",
  "term_id": "UNKNOWN:0002"
}